extrinsic component of postsynaptic endosome membrane [GO:0098999] (cellular component) Subtypes: extrinsic component of postsynaptic early endosome membrane [GO:0098998], GO:0099005 Definition: The component of the postsynaptic endosome membrane consisting of gene products and protein complexes that are loosely bound to one of its surfaces, but not integrated into the hydrophobic region. Sources: GOC:autophagy, GOC:mf Relationships: is a type of extrinsic component of endosome membrane [GO:0031313]; is part of postsynaptic endosome membrane [GO:0098895]